{
  "gene": "UniProtKB:O75366",
  "term_id": "GO:0051014",
  "gene_name": "Advillin",
  "gene_symbol": "AVIL",
  "term_label": "actin filament severing"
}